{
  "gene": "UniProtKB:O94889",
  "term_label": "cytoplasm",
  "term_id": "GO:0005737",
  "gene_name": "Kelch-like protein 18",
  "gene_symbol": "KLHL18"
}